regulation of apoptotic signaling pathway [GO:2001233] (biological process) Relationships: is_a regulation of signal transduction [GO:0009966]; is a type of GO:0042981; regulates apoptotic signaling pathway [GO:0097190] Subtypes: negative regulation of apoptotic signaling pathway [GO:2001234], GO:2001235, regulation of extrinsic apoptotic signaling pathway [GO:2001236], GO:2001242 Sources: GOC:mtg_apoptosis Also known as: regulation of apoptotic signalling pathway Definition: Any process that modulates the frequency, rate or extent of apoptotic signaling pathway.